maltose O-acetyltransferase activity [GO:0008925] (molecular function) Also known as: acetyl-CoA:maltose O-acetyltransferase activity, maltose transacetylase activity Relationships: is a type of O-acetyltransferase activity [GO:0016413] Definition: Catalysis of the reaction: acetyl-CoA + maltose = CoA + acetyl-maltose. Sources: EC:2.3.1.79